cellular response to hyperoxia [GO:0071455] (biological process) Sources: GOC:mah Definition: Any process that results in a change in state or activity of a cell (in terms of movement, secretion, enzyme production, gene expression, etc.) as a result of a stimulus indicating increased oxygen tension. Relationships: is a type of cellular response to increased oxygen levels [GO:0036295]; is a type of response to hyperoxia [GO:0055093]; is_a GO:0062197 Also known as: cellular response to hyperoxic stress, cellular response to increased oxygen tension